{
  "term_label": "cytoplasm",
  "gene": "UniProtKB:P30039",
  "term_id": "GO:0005737",
  "gene_symbol": "PBLD",
  "gene_name": "Phenazine biosynthesis-like domain-containing protein"
}